ATP-dependent chromatin remodeler activity [GO:0140658] (molecular function) Definition: An activity, driven by ATP hydrolysis, that modulates the contacts between histones and DNA, resulting in a change in chromosome architecture within the nucleosomal array, leading to chromatin remodeling. References: PMID:14729263, PMID:19165147, PMID:21862382, PMID:30867599, PMID:34313222 Also known as: ATP hydrolysis-dependent chromatin remodeler activity, ATP-dependent chromatin remodeller activity, ATPase-dependent chromatin remodeler activity, ATP-dependent chromatin remodelling, nucleosome-activated ATPase activity, nucleosome-dependent ATPase activity Relationships: is a type of ATP-dependent activity, acting on DNA [GO:0008094]; BFO_0000050 GO:0006338; has part DNA binding [GO:0003677] Subtypes: ATP-dependent histone chaperone activity [GO:0140674], histone octamer slider activity [GO:0140751]